{
  "term_id": "GO:0030174",
  "gene_symbol": "GMNC",
  "gene_name": "Geminin coiled-coil domain-containing protein 1",
  "gene": "UniProtKB:A6NCL1",
  "term_label": "regulation of DNA-templated DNA replication initiation"
}